{
  "gene_symbol": "ABCG4",
  "gene": "UniProtKB:Q9H172",
  "term_id": "GO:0055085",
  "term_label": "transmembrane transport",
  "gene_name": "ATP-binding cassette sub-family G member 4"
}